chorismate metabolic process [GO:0046417] (BP) Definition: The chemical reactions and pathways involving chorismate, the anion of (3R-trans)-3-((1-carboxyethenyl)oxy)-4-hydroxy-1,5-cyclohexadiene-1-carboxylic acid. Sources: ISBN:0198506732 Also known as: chorismate metabolism Relationships: is a type of dicarboxylic acid metabolic process [GO:0043648] Subtypes: chorismate biosynthetic process [GO:0009423], L-tyrosine biosynthetic process from chorismate via 4-hydroxyphenylpyruvate [GO:0019292], L-tyrosine biosynthetic process from chorismate via L-arogenate [GO:0033584], L-phenylalanine biosynthetic process from chorismate via phenylpyruvate [GO:0033585], L-phenylalanine biosynthetic process from chorismate via L-arogenate [GO:0033586]